{
  "gene": "UniProtKB:P31371",
  "term_id": "GO:0022008",
  "term_label": "neurogenesis",
  "gene_symbol": "FGF9",
  "gene_name": "Fibroblast growth factor 9"
}